{
  "gene": "UniProtKB:Q96IZ7",
  "term_id": "GO:0005634",
  "term_label": "nucleus",
  "gene_symbol": "RSRC1",
  "gene_name": "Serine_Arginine-related protein 53"
}